regulation of flower development [GO:0009909] (biological process) Definition: Any process that modulates the frequency, rate or extent of flower development. Sources: GOC:go_curators Subtypes: negative regulation of flower development [GO:0009910], positive regulation of flower development [GO:0009911] Relationships: is_a regulation of post-embryonic development [GO:0048580]; is a type of regulation of shoot system development [GO:0048831]; is a type of GO:2000241; regulates GO:0009908